{
  "gene": "UniProtKB:Q8NGN6",
  "gene_symbol": "OR10G7",
  "term_label": "detection of chemical stimulus involved in sensory perception of smell",
  "gene_name": "Olfactory receptor 10G7",
  "term_id": "GO:0050911"
}